{
  "term_id": "GO:0015250",
  "gene_name": "Aquaporin-4",
  "term_label": "water channel activity",
  "gene": "UniProtKB:P55087",
  "gene_symbol": "AQP4"
}